{
  "term_label": "proteasome core complex, alpha-subunit complex",
  "gene_name": "Proteasome subunit alpha-type 8",
  "term_id": "GO:0019773",
  "gene": "UniProtKB:Q8TAA3",
  "gene_symbol": "PSMA8"
}